{
  "term_id": "GO:0034355",
  "gene": "UniProtKB:Q6XQN6",
  "gene_name": "Nicotinate phosphoribosyltransferase",
  "gene_symbol": "NAPRT",
  "term_label": "NAD+ biosynthetic process via the salvage pathway"
}